{
  "gene": "UniProtKB:Q7RTY3",
  "gene_symbol": "PRSS45P",
  "gene_name": "Putative serine protease 45",
  "term_label": "proteolysis",
  "term_id": "GO:0006508"
}